{
  "term_label": "Unknown cellular component",
  "term_id": "UNKNOWN:0003",
  "gene_name": "POTE ankyrin domain family member B2",
  "gene_symbol": "POTEB2",
  "gene": "UniProtKB:H3BUK9"
}